cellular response to BMP stimulus [GO:0071773] (biological process) Sources: GOC:mah, GOC:yaf Relationships: is_a cellular response to growth factor stimulus [GO:0071363]; is a type of response to BMP [GO:0071772] Also known as: cellular response to bone morphogenetic protein stimulus Definition: Any process that results in a change in state or activity of a cell (in terms of movement, secretion, enzyme production, gene expression, etc.) as a result of a bone morphogenetic protein (BMP) stimulus.